{
  "term_label": "Unknown biological process",
  "gene_symbol": "TRAJ20",
  "gene": "UniProtKB:A0A075B6Z1",
  "gene_name": "T cell receptor alpha joining 20 (Fragment)",
  "term_id": "UNKNOWN:0002"
}